{
  "gene": "UniProtKB:Q96MM6",
  "gene_symbol": "HSPA12B",
  "gene_name": "Heat shock 70 kDa protein 12B",
  "term_id": "UNKNOWN:0002",
  "term_label": "Unknown biological process"
}